{
  "term_label": "Unknown biological process",
  "term_id": "UNKNOWN:0002",
  "gene_symbol": "RRP9",
  "gene": "UniProtKB:O43818",
  "gene_name": "U3 small nucleolar RNA-interacting protein 2"
}